{
  "gene_symbol": "G3BP1",
  "term_label": "DNA/RNA helicase activity",
  "gene": "UniProtKB:Q13283",
  "term_id": "GO:0033677",
  "gene_name": "Ras GTPase-activating protein-binding protein 1"
}